{
  "gene_symbol": "VEGFD",
  "gene_name": "Vascular endothelial growth factor D",
  "gene": "UniProtKB:O43915",
  "term_label": "vascular endothelial growth factor receptor binding",
  "term_id": "GO:0005172"
}